{
  "gene": "UniProtKB:Q8TDY2",
  "gene_name": "RB1-inducible coiled-coil protein 1",
  "term_id": "GO:0060090",
  "gene_symbol": "RB1CC1",
  "term_label": "molecular adaptor activity"
}